{
  "gene_name": "Smoothelin-like protein 1",
  "gene": "UniProtKB:A8MU46",
  "term_label": "Unknown molecular function",
  "term_id": "UNKNOWN:0001",
  "gene_symbol": "SMTNL1"
}